{
  "gene_symbol": "LRRC8E",
  "gene": "UniProtKB:Q6NSJ5",
  "term_id": "GO:0005225",
  "term_label": "volume-sensitive anion channel activity",
  "gene_name": "Volume-regulated anion channel subunit LRRC8E"
}